dynein complex binding [GO:0070840] (molecular function) Relationships: is a type of protein-containing complex binding [GO:0044877] Sources: GOC:BHF, GOC:bf, GOC:mah Definition: Binding to a dynein complex, a protein complex that contains two or three dynein heavy chains and several light chains, and has microtubule motor activity. Also known as: dynein binding